{
  "gene": "UniProtKB:P09017",
  "gene_symbol": "HOXC4",
  "term_id": "GO:0000978",
  "gene_name": "Homeobox protein Hox-C4",
  "term_label": "RNA polymerase II cis-regulatory region sequence-specific DNA binding"
}